Kdo transferase activity [GO:0043842] (molecular function) References: PMID:1577828, PMID:2033061, PMID:9195966 Definition: Catalysis of the reactions: (KDO)-lipid IVA + CMP-3-deoxy-D-manno-octulosonate = KDO2-lipid IVA + CMP, and lipid IVA + CMP-3-deoxy-D-manno-octulosonate = (KDO)-lipid IVA + CMP. Relationships: is a type of glycosyltransferase activity [GO:0016757] Also known as: 3-deoxy-D-manno-octulosonic-acid transferase activity, WaaA, kdtA